palmitic acid biosynthetic process [GO:1900535] (biological process) Relationships: is_a long-chain fatty acid biosynthetic process [GO:0042759] Definition: The chemical reactions and pathways resulting in the formation of palmitic acid. Sources: GOC:TermGenie